{
  "gene_name": "C-C motif chemokine 27",
  "gene": "UniProtKB:Q9Y4X3",
  "term_label": "chemokine activity",
  "gene_symbol": "CCL27",
  "term_id": "GO:0008009"
}